{
  "gene": "UniProtKB:O14523",
  "gene_name": "Phospholipid transfer protein C2CD2L",
  "gene_symbol": "C2CD2L",
  "term_label": "cytoplasmic side of apical plasma membrane",
  "term_id": "GO:0098592"
}